negative regulation of toll-like receptor 3 signaling pathway [GO:0034140] (biological process) Relationships: is a type of regulation of toll-like receptor 3 signaling pathway [GO:0034139]; is a type of negative regulation of cytoplasmic pattern recognition receptor signaling pathway [GO:0039532]; negatively regulates toll-like receptor 3 signaling pathway [GO:0034138] References: PMID:16551253, PMID:17328678 Sources: GOC:add Definition: Any process that stops, prevents, or reduces the frequency, rate, or extent of toll-like receptor 3 signaling pathway. Also known as: negative regulation of TLR3 signaling pathway, negative regulation of toll-like receptor 3 signalling pathway